{
  "term_id": "UNKNOWN:0003",
  "gene_symbol": "LTBR",
  "term_label": "Unknown cellular component",
  "gene_name": "Tumor necrosis factor receptor superfamily member 3",
  "gene": "UniProtKB:P36941"
}